positive regulation of androgen receptor activity [GO:2000825] (biological process) Definition: Any process that activates or increases the frequency, rate or extent of androgen receptor activity. Sources: GOC:obol Relationships: is a type of GO:0006357; is_a GO:0010469; is a type of positive regulation of DNA-binding transcription factor activity [GO:0051091]; positively regulates GO:0004879